{
  "gene_symbol": "WDR45B",
  "gene": "UniProtKB:Q5MNZ6",
  "gene_name": "WD repeat domain phosphoinositide-interacting protein 3",
  "term_id": "GO:0044804",
  "term_label": "nucleophagy"
}